{
  "gene_symbol": "C19orf67",
  "term_id": "UNKNOWN:0001",
  "gene_name": "UPF0575 protein C19orf67",
  "term_label": "Unknown molecular function",
  "gene": "UniProtKB:A6NJJ6"
}